pyruvate transport [GO:0006848] (biological process) Subtypes: pyruvate transmembrane transport [GO:1901475] Relationships: is a type of GO:0015718 Definition: The directed movement of pyruvate into, out of or within a cell, or between cells, by means of some agent such as a transporter or pore. Sources: GOC:krc